{
  "gene": "UniProtKB:Q9NWV4",
  "term_id": "GO:0008270",
  "gene_name": "CXXC motif containing zinc binding protein",
  "gene_symbol": "CZIB",
  "term_label": "zinc ion binding"
}